{
  "gene_symbol": "CRYAA",
  "gene": "UniProtKB:P02489",
  "gene_name": "Alpha-crystallin A chain",
  "term_label": "nucleus",
  "term_id": "GO:0005634"
}